{
  "gene": "UniProtKB:Q8WXJ9",
  "term_id": "UNKNOWN:0003",
  "gene_name": "Ankyrin repeat and SOCS box protein 17",
  "term_label": "Unknown cellular component",
  "gene_symbol": "ASB17"
}